{
  "gene": "UniProtKB:P01742",
  "gene_symbol": "IGHV1-69",
  "gene_name": "Immunoglobulin heavy variable 1-69",
  "term_id": "GO:0016064",
  "term_label": "immunoglobulin mediated immune response"
}